{
  "term_id": "GO:0034504",
  "gene_name": "Glucokinase regulatory protein",
  "term_label": "protein localization to nucleus",
  "gene_symbol": "GCKR",
  "gene": "UniProtKB:Q14397"
}